positive regulation of mating type switching [GO:0031496] (biological process) Sources: GOC:mah Relationships: is a type of regulation of mating type switching [GO:0031494]; is a type of positive regulation of developmental process [GO:0051094]; is a type of positive regulation of reproductive process [GO:2000243]; positively regulates mating type switching [GO:0007533] Also known as: up regulation of mating type switching, up-regulation of mating type switching, upregulation of mating type switching, activation of mating type switching, stimulation of mating type switching Definition: Any process that activates or increases the frequency, rate or extent of mating type switching.